{
  "gene": "UniProtKB:Q8N434",
  "term_id": "UNKNOWN:0003",
  "term_label": "Unknown cellular component",
  "gene_name": "Putative transporter SVOPL",
  "gene_symbol": "SVOPL"
}